{
  "term_id": "UNKNOWN:0001",
  "gene_name": "SLAM family member 7",
  "gene_symbol": "SLAMF7",
  "term_label": "Unknown molecular function",
  "gene": "UniProtKB:Q9NQ25"
}